{
  "gene_symbol": "DEFB133",
  "term_label": "CCR6 chemokine receptor binding",
  "term_id": "GO:0031731",
  "gene_name": "Beta-defensin 133",
  "gene": "UniProtKB:Q30KQ1"
}